{
  "term_id": "GO:0030150",
  "gene": "UniProtKB:Q9Y5T4",
  "term_label": "protein import into mitochondrial matrix",
  "gene_symbol": "DNAJC15",
  "gene_name": "DnaJ homolog subfamily C member 15"
}